{
  "gene_symbol": "PHTF2",
  "gene_name": "Protein PHTF2",
  "gene": "UniProtKB:Q8N3S3",
  "term_id": "UNKNOWN:0001",
  "term_label": "Unknown molecular function"
}